{
  "gene_name": "Putative transmembrane protein 217B",
  "gene": "UniProtKB:A0A494BZU4",
  "term_label": "Unknown molecular function",
  "term_id": "UNKNOWN:0001",
  "gene_symbol": "TMEM217B"
}